{
  "term_id": "UNKNOWN:0002",
  "gene_symbol": "LCN10",
  "term_label": "Unknown biological process",
  "gene": "UniProtKB:Q6JVE6",
  "gene_name": "Epididymal-specific lipocalin-10"
}